amylin receptor complex 3 [GO:0150058] (cellular component) Definition: A G protein-coupled receptor complex that serves as a receptor for amylin polypeptide (AMY) and consists of a calcitonin receptor (CTR/CALCR) and a receptor activity-modifying protein (RAMP) 3. Amylin receptor complex 3 (AMY3) also serves as a receptor for the amyloid-beta complex. Ligand binding to AMY3 results in increased cytosolic calcium ion levels and in activation on multiple intracellular signaling pathways. References: PMID:22500019 Sources: GOC:aruk, GOC:bc Also known as: AMY3 complex Relationships: is a type of amylin receptor complex [GO:1903440]